{
  "gene_symbol": "TYRP1",
  "term_label": "melanosome organization",
  "gene": "UniProtKB:P17643",
  "gene_name": "5,6-dihydroxyindole-2-carboxylic acid oxidase",
  "term_id": "GO:0032438"
}